{
  "term_label": "Unknown cellular component",
  "term_id": "UNKNOWN:0003",
  "gene_name": "ATP synthase F(0) complex subunit B1, mitochondrial",
  "gene": "UniProtKB:P24539",
  "gene_symbol": "ATP5PB"
}